{
  "gene": "UniProtKB:Q9UHG0",
  "term_label": "microtubule",
  "gene_symbol": "DCDC2",
  "term_id": "GO:0005874",
  "gene_name": "Doublecortin domain-containing protein 2"
}